{
  "term_label": "nucleus",
  "term_id": "GO:0005634",
  "gene": "UniProtKB:Q5T6S3",
  "gene_name": "PHD finger protein 19",
  "gene_symbol": "PHF19"
}